{
  "gene_symbol": "SBDS",
  "term_label": "Unknown biological process",
  "gene_name": "Ribosome maturation protein SBDS",
  "term_id": "UNKNOWN:0002",
  "gene": "UniProtKB:Q9Y3A5"
}